{
  "term_id": "GO:0004757",
  "gene_symbol": "SPR",
  "gene": "UniProtKB:P35270",
  "gene_name": "Sepiapterin reductase",
  "term_label": "sepiapterin reductase (NADP+) activity"
}